negative regulation of phosphatidylglycerol biosynthetic process [GO:1901352] (biological process) References: PMID:12869188 Sources: GOC:TermGenie, GOC:dgf Also known as: down regulation of phosphatidylglycerol anabolism, down regulation of phosphatidylglycerol biosynthesis, down regulation of phosphatidylglycerol biosynthetic process, down regulation of phosphatidylglycerol formation, down regulation of phosphatidylglycerol synthesis, down-regulation of phosphatidylglycerol anabolism, down-regulation of phosphatidylglycerol biosynthesis, down-regulation of phosphatidylglycerol biosynthetic process, down-regulation of phosphatidylglycerol formation, down-regulation of phosphatidylglycerol synthesis, downregulation of phosphatidylglycerol anabolism, downregulation of phosphatidylglycerol biosynthesis, downregulation of phosphatidylglycerol biosynthetic process, downregulation of phosphatidylglycerol formation, downregulation of phosphatidylglycerol synthesis, negative regulation of phosphatidylglycerol anabolism, negative regulation of phosphatidylglycerol biosynthesis, negative regulation of phosphatidylglycerol formation, negative regulation of phosphatidylglycerol synthesis, inhibition of phosphatidylglycerol anabolism, inhibition of phosphatidylglycerol biosynthesis, inhibition of phosphatidylglycerol biosynthetic process, inhibition of phosphatidylglycerol formation, inhibition of phosphatidylglycerol synthesis Relationships: is a type of negative regulation of phospholipid biosynthetic process [GO:0071072]; is a type of regulation of phosphatidylglycerol biosynthetic process [GO:1901351]; RO_0002212 GO:0006655 Definition: Any process that stops, prevents or reduces the frequency, rate or extent of phosphatidylglycerol biosynthetic process.